{
  "gene_symbol": "FOXN2",
  "term_label": "regulation of DNA-templated transcription",
  "term_id": "GO:0006355",
  "gene_name": "Forkhead box protein N2",
  "gene": "UniProtKB:P32314"
}